{
  "term_label": "glial cell-derived neurotrophic factor receptor signaling pathway",
  "gene_name": "Glial cell line-derived neurotrophic factor",
  "gene_symbol": "GDNF",
  "term_id": "GO:0035860",
  "gene": "UniProtKB:P39905"
}